{
  "term_id": "GO:0000981",
  "gene_name": "Homeobox protein Hox-B6",
  "term_label": "DNA-binding transcription factor activity, RNA polymerase II-specific",
  "gene": "UniProtKB:P17509",
  "gene_symbol": "HOXB6"
}